{
  "gene_symbol": "ATP1B1",
  "gene_name": "Sodium_potassium-transporting ATPase subunit beta-1",
  "gene": "UniProtKB:P05026",
  "term_id": "GO:0006883",
  "term_label": "intracellular sodium ion homeostasis"
}